beta-D-galactofuranose biosynthetic process [GO:1901358] (biological process) Definition: The chemical reactions and pathways resulting in the formation of beta-D-galactofuranose. Sources: GOC:TermGenie, GOC:di Also known as: beta-D-galactofuranose anabolism, beta-D-galactofuranose biosynthesis, beta-D-galactofuranose formation, beta-D-galactofuranose synthesis Relationships: is a type of galactose biosynthetic process [GO:0046369]